{
  "term_label": "RNA polymerase II cis-regulatory region sequence-specific DNA binding",
  "term_id": "GO:0000978",
  "gene_name": "Zinc finger protein 880",
  "gene": "UniProtKB:Q6PDB4",
  "gene_symbol": "ZNF880"
}